{
  "gene_name": "Spermatogenesis-associated protein 9",
  "gene_symbol": "SPATA9",
  "term_label": "Unknown molecular function",
  "term_id": "UNKNOWN:0001",
  "gene": "UniProtKB:Q9BWV2"
}